posterior lateral line ganglion development [GO:0048917] (BP) Definition: The process whose specific outcome is the progression of the posterior lateral line ganglion over time, from its formation to the mature structure. The posterior lateral line ganglion develops from cranial ectodermal placodes situated behind the ear. Sources: ISBN:0125296509, ISBN:0387968377 Also known as: gPLL development Relationships: is a type of GO:0048890; is part of posterior lateral line system development [GO:0048915]